{
  "term_id": "UNKNOWN:0002",
  "gene": "UniProtKB:Q58A44",
  "term_label": "Unknown biological process",
  "gene_symbol": "PCOTH",
  "gene_name": "Prostate collagen triple helix protein"
}